{
  "gene_name": "Sphingosine 1-phosphate receptor 1",
  "gene_symbol": "S1PR1",
  "term_label": "angiogenesis",
  "term_id": "GO:0001525",
  "gene": "UniProtKB:P21453"
}